{
  "gene_name": "Protein spire homolog 1",
  "term_label": "cell cortex",
  "gene": "UniProtKB:Q08AE8",
  "term_id": "GO:0005938",
  "gene_symbol": "SPIRE1"
}